{
  "gene_name": "Isobutyryl-CoA dehydrogenase, mitochondrial",
  "term_id": "UNKNOWN:0002",
  "gene": "UniProtKB:Q9UKU7",
  "term_label": "Unknown biological process",
  "gene_symbol": "ACAD8"
}